kidney vasculature development [GO:0061440] (biological process) Subtypes: glomerulus vasculature development [GO:0072012] Definition: The process whose specific outcome is the progression of the vasculature of the kidney over time, from its formation to the mature structure. References: PMID:11891195 Sources: GOC:dph, GOC:mtg_kidney_jan10 Relationships: is a type of renal system vasculature development [GO:0061437]; BFO_0000050 GO:0001822